bile acid metabolic process [GO:0008206] (biological process) Definition: The chemical reactions and pathways involving bile acids, a group of steroid carboxylic acids occurring in bile, where they are present as the sodium salts of their amides with glycine or taurine. Sources: GOC:go_curators Relationships: is a type of steroid metabolic process [GO:0008202]; is a type of monocarboxylic acid metabolic process [GO:0032787] Subtypes: bile acid conjugation [GO:0002152], GO:0006699, bile acid catabolic process [GO:0030573] Also known as: bile acid metabolism